{
  "gene_symbol": "TAF6L",
  "term_id": "GO:0003713",
  "term_label": "transcription coactivator activity",
  "gene": "UniProtKB:Q9Y6J9",
  "gene_name": "TAF6-like RNA polymerase II p300_CBP-associated factor-associated factor 65 kDa subunit 6L"
}